regulation of bicoid mRNA localization [GO:0008359] (biological process) Subtypes: negative regulation of bicoid mRNA localization [GO:0045853], positive regulation of bicoid mRNA localization [GO:0045854] Definition: Any process that modulates the frequency, rate or extent of the process in which bicoid mRNA is transported to, or maintained in, a specific location. Also known as: regulation of bicoid mRNA localisation Sources: GOC:hb Relationships: is a type of regulation of intracellular mRNA localization [GO:1904580]; regulates GO:0045450